{
  "gene": "UniProtKB:Q8N5H7",
  "term_id": "UNKNOWN:0001",
  "gene_name": "SH2 domain-containing protein 3C",
  "gene_symbol": "SH2D3C",
  "term_label": "Unknown molecular function"
}